{
  "gene": "UniProtKB:Q8IWP9",
  "term_id": "UNKNOWN:0001",
  "gene_symbol": "CCDC28A",
  "gene_name": "Coiled-coil domain-containing protein 28A",
  "term_label": "Unknown molecular function"
}